{
  "gene_symbol": "FRYL",
  "term_label": "Unknown molecular function",
  "gene_name": "Protein furry homolog-like",
  "gene": "UniProtKB:O94915",
  "term_id": "UNKNOWN:0001"
}